{
  "gene_name": "Uncharacterized protein C5orf47",
  "term_id": "UNKNOWN:0003",
  "gene": "UniProtKB:Q569G3",
  "gene_symbol": "C5orf47",
  "term_label": "Unknown cellular component"
}